positive regulation of endothelial cell chemotaxis [GO:2001028] (biological process) Relationships: is a type of positive regulation of endothelial cell migration [GO:0010595]; is a type of GO:0050921; is a type of regulation of endothelial cell chemotaxis [GO:2001026]; positively regulates GO:0035767 Definition: Any process that activates or increases the frequency, rate or extent of endothelial cell chemotaxis. Subtypes: GO:0038033, positive regulation of endothelial cell chemotaxis to fibroblast growth factor [GO:2000546] Sources: GOC:BHF